{
  "gene": "UniProtKB:Q9H1R2",
  "term_label": "protein tyrosine phosphatase activity",
  "gene_symbol": "DUSP15",
  "term_id": "GO:0004725",
  "gene_name": "Dual specificity protein phosphatase 15"
}